{
  "gene": "UniProtKB:Q53S08",
  "term_label": "retrograde vesicle-mediated transport, Golgi to endoplasmic reticulum",
  "gene_name": "Ras-related protein Rab-6D",
  "gene_symbol": "RAB6D",
  "term_id": "GO:0006890"
}